{
  "gene_name": "Recombining binding protein suppressor of hairless-like protein",
  "gene": "UniProtKB:Q9UBG7",
  "term_id": "GO:0000981",
  "term_label": "DNA-binding transcription factor activity, RNA polymerase II-specific",
  "gene_symbol": "RBPJL"
}